regulation of lymphocyte differentiation [GO:0045619] (biological process) Definition: Any process that modulates the frequency, rate or extent of lymphocyte differentiation. Note: Note that immunologists typically use the word 'development' to refer to cells of B or T cell lineages undergoing the process that GO describes as 'cell differentiation'. Sources: GOC:go_curators Also known as: regulation of lymphocyte development Relationships: is a type of regulation of lymphocyte activation [GO:0051249]; is a type of regulation of leukocyte differentiation [GO:1902105]; regulates lymphocyte differentiation [GO:0030098] Subtypes: regulation of natural killer cell differentiation [GO:0032823], regulation of B cell differentiation [GO:0045577], regulation of T cell differentiation [GO:0045580], negative regulation of lymphocyte differentiation [GO:0045620], GO:0045621